{
  "term_label": "mitochondrion",
  "gene_symbol": "NME6",
  "gene": "UniProtKB:O75414",
  "gene_name": "Nucleoside diphosphate kinase 6",
  "term_id": "GO:0005739"
}